{
  "term_label": "chaperonin-containing T-complex",
  "gene": "UniProtKB:P17987",
  "gene_symbol": "TCP1",
  "gene_name": "T-complex protein 1 subunit alpha",
  "term_id": "GO:0005832"
}